{
  "term_label": "TORC1 complex",
  "term_id": "GO:0031931",
  "gene_symbol": "RPTOR",
  "gene_name": "Regulatory-associated protein of mTOR",
  "gene": "UniProtKB:Q8N122"
}